{
  "gene_name": "Membrane-associated transporter protein",
  "term_id": "GO:0048066",
  "gene_symbol": "SLC45A2",
  "term_label": "developmental pigmentation",
  "gene": "UniProtKB:Q9UMX9"
}